{
  "term_id": "GO:0033700",
  "gene_symbol": "APOA5",
  "term_label": "phospholipid efflux",
  "gene_name": "Apolipoprotein A-V",
  "gene": "UniProtKB:Q6Q788"
}